{
  "gene": "UniProtKB:O60890",
  "term_id": "GO:0005096",
  "gene_symbol": "OPHN1",
  "term_label": "GTPase activator activity",
  "gene_name": "Oligophrenin-1"
}